{
  "gene_symbol": "ESRRA",
  "gene": "UniProtKB:P11474",
  "term_label": "chromatin",
  "term_id": "GO:0000785",
  "gene_name": "Steroid hormone receptor ERR1"
}